{
  "gene_name": "Solute carrier family 12 member 3",
  "gene": "UniProtKB:P55017",
  "term_id": "GO:1902476",
  "term_label": "chloride transmembrane transport",
  "gene_symbol": "SLC12A3"
}